{
  "gene_symbol": "NEXMIF",
  "gene": "UniProtKB:Q5QGS0",
  "term_label": "negative regulation of cell adhesion mediated by integrin",
  "gene_name": "Neurite extension and migration factor",
  "term_id": "GO:0033629"
}